formate metabolic process [GO:0015942] (biological process) Also known as: formate metabolism Sources: ISBN:0198506732 Definition: The chemical reactions and pathways involving formate, also known as methanoate, the anion HCOO- derived from methanoic (formic) acid. Subtypes: formate biosynthetic process [GO:0015943], formate oxidation [GO:0015944], L-histidine catabolic process to glutamate and formate [GO:0019557], creatinine catabolic process to formate [GO:0019621], mixed acid fermentation [GO:0019664], formate catabolic process [GO:0042183], methane biosynthetic process from formic acid [GO:2001127] Relationships: is a type of monocarboxylic acid metabolic process [GO:0032787]